{
  "gene_symbol": "CTSG",
  "term_id": "GO:0004252",
  "gene_name": "Cathepsin G",
  "gene": "UniProtKB:P08311",
  "term_label": "serine-type endopeptidase activity"
}